{
  "gene": "UniProtKB:Q9H0P7",
  "gene_symbol": "AGPAT4-IT1",
  "term_label": "Unknown cellular component",
  "term_id": "UNKNOWN:0003",
  "gene_name": "Putative uncharacterized protein encoded by AGPAT4-IT1"
}